{
  "term_id": "GO:0038023",
  "gene_symbol": "ITGA8",
  "gene": "UniProtKB:P53708",
  "gene_name": "Integrin alpha-8",
  "term_label": "signaling receptor activity"
}